{
  "term_id": "GO:1904263",
  "gene_name": "Ras-related GTP-binding protein C",
  "gene": "UniProtKB:Q9HB90",
  "gene_symbol": "RRAGC",
  "term_label": "positive regulation of TORC1 signaling"
}